{
  "gene_name": "Actin-related protein 2_3 complex subunit 1B",
  "term_id": "UNKNOWN:0001",
  "term_label": "Unknown molecular function",
  "gene": "UniProtKB:O15143",
  "gene_symbol": "ARPC1B"
}